{
  "gene_name": "LIM and senescent cell antigen-like-containing domain protein 1",
  "gene_symbol": "LIMS1",
  "gene": "UniProtKB:P48059",
  "term_id": "GO:2001046",
  "term_label": "positive regulation of integrin-mediated signaling pathway"
}